{
  "gene_symbol": "KRTAP9-6",
  "term_label": "Unknown biological process",
  "gene": "UniProtKB:A0A140TA67",
  "gene_name": "Keratin-associated protein 9-6",
  "term_id": "UNKNOWN:0002"
}